{
  "gene_name": "Sphingosine 1-phosphate receptor 3",
  "term_label": "plasma membrane",
  "gene": "UniProtKB:Q99500",
  "gene_symbol": "S1PR3",
  "term_id": "GO:0005886"
}